{
  "gene_name": "1-phosphatidylinositol 4,5-bisphosphate phosphodiesterase delta-3",
  "gene_symbol": "PLCD3",
  "term_id": "UNKNOWN:0002",
  "gene": "UniProtKB:Q8N3E9",
  "term_label": "Unknown biological process"
}